{
  "term_label": "behavioral response to starvation",
  "term_id": "GO:0042595",
  "gene": "UniProtKB:Q9UBC7",
  "gene_name": "Galanin-like peptide",
  "gene_symbol": "GALP"
}